negative regulation of clathrin coat assembly [GO:1905444] (biological process) Definition: Any process that stops, prevents or reduces the frequency, rate or extent of clathrin coat assembly. Sources: GOC:PARL, GOC:TermGenie, GOC:bf, GO_REF:0000058 Also known as: down regulation of clathrin cage assembly, down regulation of clathrin coat assembly, down-regulation of clathrin cage assembly, down-regulation of clathrin coat assembly, downregulation of clathrin cage assembly, downregulation of clathrin coat assembly, negative regulation of clathrin cage assembly, inhibition of clathrin cage assembly, inhibition of clathrin coat assembly Relationships: is a type of negative regulation of protein-containing complex assembly [GO:0031333]; is a type of regulation of clathrin coat assembly [GO:1905443]; negatively regulates clathrin coat assembly [GO:0048268]